{
  "term_id": "GO:0005829",
  "gene_name": "Probable ubiquitin carboxyl-terminal hydrolase FAF-X",
  "gene": "UniProtKB:Q93008",
  "term_label": "cytosol",
  "gene_symbol": "USP9X"
}